{
  "term_label": "Unknown biological process",
  "term_id": "UNKNOWN:0002",
  "gene_name": "AP-4 complex subunit epsilon-1",
  "gene_symbol": "AP4E1",
  "gene": "UniProtKB:Q9UPM8"
}